{
  "gene": "UniProtKB:P05106",
  "gene_name": "Integrin beta-3",
  "gene_symbol": "ITGB3",
  "term_label": "cell adhesion mediated by integrin",
  "term_id": "GO:0033627"
}